NAD(P)+ transhydrogenase (Si-specific) activity [GO:0003957] (molecular function) Relationships: is a type of oxidoreductase activity, acting on NAD(P)H as acceptor [GO:0016652] Also known as: H+-thase, NAD transhydrogenase, NADH transhydrogenase, NADH-NADP-transhydrogenase, NADPH-NAD oxidoreductase, NADPH-NAD transhydrogenase, NADPH:NAD+ transhydrogenase, nicotinamide adenine dinucleotide (phosphate) transhydrogenase, nicotinamide nucleotide transhydrogenase activity, pyridine nucleotide transferase, pyridine nucleotide transhydrogenase activity, NAD(P) transhydrogenase (B-specific) activity, NAD(P)+ transhydrogenase (B-specific) activity, NADPH:NAD+ oxidoreductase (B-specific), non-energy-linked transhydrogenase activity Sources: RHEA:11692 Definition: Catalysis of the reaction: NADPH + NAD+ = NADP+ + NADH.